calcium:manganese antiporter activity [GO:0140983] (MF) Relationships: is a type of manganese ion transmembrane transporter activity [GO:0005384]; is a type of GO:0015368 Definition: Catalysis of the reaction: Ca2+(in) + Mn2+(out) = Ca2+(out) + Mn2+(in). Also known as: manganese:calcium antiporter activity References: PMID:30755481